{
  "gene_symbol": "GPAT4",
  "gene": "UniProtKB:Q86UL3",
  "gene_name": "Glycerol-3-phosphate acyltransferase 4",
  "term_id": "UNKNOWN:0002",
  "term_label": "Unknown biological process"
}